{
  "term_label": "DNA-binding transcription factor activity, RNA polymerase II-specific",
  "gene_symbol": "HOXD4",
  "gene": "UniProtKB:P09016",
  "term_id": "GO:0000981",
  "gene_name": "Homeobox protein Hox-D4"
}